{
  "gene": "UniProtKB:Q8IW41",
  "term_id": "GO:0005634",
  "term_label": "nucleus",
  "gene_symbol": "MAPKAPK5",
  "gene_name": "MAP kinase-activated protein kinase 5"
}